platelet-derived growth factor alpha-receptor activity [GO:0005018] (molecular function) Definition: Combining with platelet-derived growth factor isoform PDGF-AA, PDGF-BB or PDGF-AB to initiate a change in cell activity. Relationships: is a type of platelet-derived growth factor receptor activity [GO:0005017]; is part of platelet-derived growth factor receptor-alpha signaling pathway [GO:0035790] References: PMID:1657917 Also known as: PDGF alpha-receptor activity, alphaPDGF receptor activity